stevioside glucosyltransferase activity (rebaudioside A forming) [GO:0102381] (molecular function) Definition: Catalysis of the reaction: stevioside + UDP-alpha-D-glucose = H+ + rebaudioside A + UDP. Sources: RHEA:61756 Relationships: is a type of hexosyltransferase activity [GO:0016758]